tricarboxylate secondary active transmembrane transporter activity [GO:0005371] (molecular function) Also known as: tricarboxylate carrier activity Definition: Enables the transfer of tricarboxylate from one side of a membrane to the other, up its concentration gradient. The transporter binds the solute and undergoes a series of conformational changes. Transport works equally well in either direction and is driven by a chemiosmotic source of energy. Secondary active transporters include symporters and antiporters. Sources: GOC:mtg_transport, ISBN:0815340729 Relationships: is a type of secondary active transmembrane transporter activity [GO:0015291]; is a type of carboxylic acid transmembrane transporter activity [GO:0046943] Subtypes: citrate secondary active transmembrane transporter activity [GO:0071913]